term replaced by [IAO:0100001]